{
  "gene_symbol": "TRGJP",
  "term_id": "UNKNOWN:0002",
  "gene_name": "T cell receptor gamma joining P (Fragment)",
  "gene": "UniProtKB:A0A0C4DH63",
  "term_label": "Unknown biological process"
}